{
  "gene_symbol": "ADAMTSL4-AS1",
  "gene_name": "Uncharacterized protein ADAMTSL4-AS1",
  "gene": "UniProtKB:Q5T5F5",
  "term_label": "Unknown biological process",
  "term_id": "UNKNOWN:0002"
}